anterograde axonal transport of messenger ribonucleoprotein complex [GO:0099087] (biological process) References: PMID:26586091 Sources: GOC:dos Also known as: anterograde axonal transport of mRNA RNP complex Relationships: is_a anterograde axonal transport [GO:0008089] Definition: The directed movement of a messenger ribonucleoprotein complex along microtubules in axons, towards the presynapse.